{
  "gene": "UniProtKB:Q7Z434",
  "gene_name": "Mitochondrial antiviral-signaling protein",
  "term_id": "UNKNOWN:0002",
  "gene_symbol": "MAVS",
  "term_label": "Unknown biological process"
}